{
  "term_label": "nucleus",
  "gene": "UniProtKB:Q04743",
  "gene_name": "Homeobox protein EMX2",
  "term_id": "GO:0005634",
  "gene_symbol": "EMX2"
}